{
  "term_label": "negative regulation of complement activation, alternative pathway",
  "gene": "UniProtKB:Q9Y279",
  "term_id": "GO:0045957",
  "gene_symbol": "VSIG4",
  "gene_name": "V-set and immunoglobulin domain-containing protein 4"
}